{
  "term_label": "cytoplasm",
  "gene_symbol": "VIPAS39",
  "gene_name": "Spermatogenesis-defective protein 39 homolog",
  "term_id": "GO:0005737",
  "gene": "UniProtKB:Q9H9C1"
}